{
  "term_id": "GO:0007265",
  "gene_name": "Rap guanine nucleotide exchange factor 5",
  "term_label": "Ras protein signal transduction",
  "gene": "UniProtKB:Q92565",
  "gene_symbol": "RAPGEF5"
}